{
  "gene_symbol": "ZNF714",
  "term_label": "DNA-binding transcription factor activity, RNA polymerase II-specific",
  "gene_name": "Zinc finger protein 714",
  "term_id": "GO:0000981",
  "gene": "UniProtKB:Q96N38"
}